negative regulation of cholesterol storage [GO:0010887] (biological process) Also known as: negative regulation of cholesterol sequestration Sources: GOC:BHF, GOC:dph, GOC:tb Relationships: is a type of regulation of cholesterol storage [GO:0010885]; is a type of negative regulation of lipid storage [GO:0010888]; negatively regulates cholesterol storage [GO:0010878] Definition: Any process that decreases the rate or extent of cholesterol storage. Cholesterol storage is the accumulation and maintenance in cells or tissues of cholesterol, cholest-5-en-3 beta-ol, the principal sterol of vertebrates and the precursor of many steroids, including bile acids and steroid hormones.